{
  "gene_symbol": "PAXIP1",
  "gene": "UniProtKB:Q6ZW49",
  "term_label": "DNA damage response",
  "gene_name": "PAX-interacting protein 1",
  "term_id": "GO:0006974"
}